{
  "gene_name": "Proto-oncogene Wnt-3",
  "term_id": "GO:0030182",
  "term_label": "neuron differentiation",
  "gene_symbol": "WNT3",
  "gene": "UniProtKB:P56703"
}